type IV hypersensitivity [GO:0001806] (biological process) Relationships: is a type of GO:0002456; is a type of hypersensitivity [GO:0002524] Regulation: RO_0002211 by regulation of type IV hypersensitivity [GO:0001807]; negatively regulated by GO:0001808; RO_0002213 by positive regulation of type IV hypersensitivity [GO:0001809] Definition: An inflammatory response driven by T cell recognition of processed soluble or cell-associated antigens leading to cytokine release and leukocyte activation. Sources: GOC:add, ISBN:0781735149 Also known as: delayed hypersensitivity response, delayed-type hypersensitivity